vascular process in circulatory system [GO:0003018] (biological process) Also known as: vasculature process Relationships: is_a circulatory system process [GO:0003013] Definition: A circulatory process that occurs at the level of the vasculature. Subtypes: baroreceptor detection of arterial stretch [GO:0001981], vascular transport [GO:0010232], GO:0043114, blood vessel diameter maintenance [GO:0097746], lymphatic vascular process in circulatory system [GO:1990183] Sources: GOC:mtg_cardio